{
  "gene": "UniProtKB:Q9NVS9",
  "gene_symbol": "PNPO",
  "term_label": "pyridoxamine phosphate oxidase activity",
  "term_id": "GO:0004733",
  "gene_name": "Pyridoxine-5'-phosphate oxidase"
}